{
  "gene": "UniProtKB:P25789",
  "term_label": "proteasome-mediated ubiquitin-dependent protein catabolic process",
  "gene_name": "Proteasome subunit alpha type-4",
  "term_id": "GO:0043161",
  "gene_symbol": "PSMA4"
}